{
  "gene": "UniProtKB:P08572",
  "gene_name": "Collagen alpha-2(IV) chain",
  "term_label": "extracellular matrix organization",
  "term_id": "GO:0030198",
  "gene_symbol": "COL4A2"
}